{
  "gene_name": "Zinc finger protein 141",
  "term_label": "DNA-binding transcription factor activity, RNA polymerase II-specific",
  "gene": "UniProtKB:Q15928",
  "term_id": "GO:0000981",
  "gene_symbol": "ZNF141"
}